{
  "gene_symbol": "NCCRP1",
  "gene_name": "F-box only protein 50",
  "term_id": "GO:0036503",
  "term_label": "ERAD pathway",
  "gene": "UniProtKB:Q6ZVX7"
}